{
  "term_label": "RNA polymerase II cis-regulatory region sequence-specific DNA binding",
  "term_id": "GO:0000978",
  "gene": "UniProtKB:P43699",
  "gene_name": "Homeobox protein Nkx-2.1",
  "gene_symbol": "NKX2-1"
}